{
  "gene_name": "Probable global transcription activator SNF2L2",
  "gene_symbol": "SMARCA2",
  "term_label": "heterochromatin formation",
  "term_id": "GO:0031507",
  "gene": "UniProtKB:P51531"
}